{
  "term_id": "GO:0031175",
  "gene_symbol": "STMN3",
  "gene_name": "Stathmin-3",
  "gene": "UniProtKB:Q9NZ72",
  "term_label": "neuron projection development"
}